neurexin clustering involved in presynaptic membrane assembly [GO:0097115] (biological process) Definition: The receptor clustering process involved in assembly of the presynaptic membrane in which neurexins are localized to distinct domains in the cell membrane. Neurexins are synaptic cell surface proteins which act as cell recognition molecules at nerve terminals. Relationships: is a type of GO:0043113; is part of presynaptic membrane assembly [GO:0097105] Also known as: Nrxn clustering, neurexin clustering, presynaptic neurexin clustering References: PMID:12796785 Sources: GOC:BHF, GOC:sjp